{
  "term_id": "GO:0010265",
  "gene_name": "Cullin-associated NEDD8-dissociated protein 1",
  "gene_symbol": "CAND1",
  "gene": "UniProtKB:Q86VP6",
  "term_label": "SCF complex assembly"
}